{
  "term_id": "GO:0030947",
  "gene_name": "Hypoxia-inducible factor 1-alpha inhibitor",
  "gene": "UniProtKB:Q9NWT6",
  "term_label": "regulation of vascular endothelial growth factor receptor signaling pathway",
  "gene_symbol": "HIF1AN"
}